{
  "gene_symbol": "OR2A12",
  "gene": "UniProtKB:Q8NGT7",
  "gene_name": "Olfactory receptor 2A12",
  "term_id": "GO:0004984",
  "term_label": "olfactory receptor activity"
}